{
  "gene": "UniProtKB:Q86XG9",
  "term_label": "Unknown biological process",
  "term_id": "UNKNOWN:0002",
  "gene_name": "Putative neuroblastoma breakpoint family member 5",
  "gene_symbol": "NBPF5P"
}